kidney field specification [GO:0072004] (biological process) Also known as: specification of kidney anlage Definition: The process that results in the delineation of regions of the embryo into the area in which the kidney rudiment will develop. Sources: GOC:mtg_kidney_jan10 Relationships: is a type of specification of animal organ identity [GO:0010092]; is_a GO:0061004; is part of kidney rudiment formation [GO:0072003] Subtypes: GO:0039003